{
  "gene_symbol": "STAU2",
  "term_id": "GO:0098964",
  "gene_name": "Double-stranded RNA-binding protein Staufen homolog 2",
  "term_label": "anterograde dendritic transport of messenger ribonucleoprotein complex",
  "gene": "UniProtKB:Q9NUL3"
}